{
  "gene_symbol": "PAN2",
  "gene_name": "PAN2-PAN3 deadenylation complex catalytic subunit PAN2",
  "term_label": "Unknown molecular function",
  "gene": "UniProtKB:Q504Q3",
  "term_id": "UNKNOWN:0001"
}